{
  "term_id": "GO:0005886",
  "term_label": "plasma membrane",
  "gene_name": "Muscle, skeletal receptor tyrosine-protein kinase",
  "gene": "UniProtKB:O15146",
  "gene_symbol": "MUSK"
}